{
  "gene_name": "Metallothionein-1A",
  "gene": "UniProtKB:P04731",
  "gene_symbol": "MT1A",
  "term_label": "cellular response to zinc ion",
  "term_id": "GO:0071294"
}